maintenance of gastrointestinal epithelium [GO:0030277] (biological process) Definition: Protection of epithelial surfaces of the gastrointestinal tract from proteolytic and caustic digestive agents. Relationships: is a type of GO:0010669; is_a digestive system process [GO:0022600] Subtypes: GO:0060729 Sources: GOC:mah